Z granule [GO:0120279] (cellular component) References: PMID:29769721, PMID:31378614, PMID:32650583 Sources: GOC:dr, GOC:krc Definition: A small cytoplasmic, non-membranous RNA/protein complex aggregate in the primordial germ cells that are distinct from, but colocalize with or are adjacent to, P granules and mutator foci and are associated with RNA metabolism. Z granules have been observed in C. elegans. Also known as: germline granule Relationships: is a type of cytoplasmic ribonucleoprotein granule [GO:0036464]; is part of germ plasm [GO:0060293]